{
  "gene_name": "Stathmin domain-containing protein 1",
  "gene_symbol": "STMND1",
  "term_label": "regulation of microtubule polymerization or depolymerization",
  "gene": "UniProtKB:H3BQB6",
  "term_id": "GO:0031110"
}